{
  "gene": "UniProtKB:Q9H1K6",
  "term_label": "Unknown cellular component",
  "gene_name": "Talin rod domain-containing protein 1",
  "term_id": "UNKNOWN:0003",
  "gene_symbol": "TLNRD1"
}